{
  "term_label": "ATP hydrolysis activity",
  "gene_symbol": "VCP",
  "gene_name": "Transitional endoplasmic reticulum ATPase",
  "gene": "UniProtKB:P55072",
  "term_id": "GO:0016887"
}